{
  "gene_name": "Peroxisomal membrane protein PEX13",
  "gene_symbol": "PEX13",
  "term_label": "Unknown molecular function",
  "gene": "UniProtKB:Q92968",
  "term_id": "UNKNOWN:0001"
}